transposable element silencing by piRNA-mediated DNA methylation [GO:0141196] (biological process) Relationships: is a type of GO:0141005; is a type of gene silencing by piRNA-directed DNA methylation [GO:0141176] Also known as: transposable element silencing by piRNA-directed DNA methylation, retrotransposon silencing by piRNA-directed DNA methylation Definition: A transposable element silencing mechanism mediated by Piwi-associated RNA (piRNA)-directed DNA methylation. This results in a heterochromatin assembly, a chromatin conformation that is refractory to transcription. References: PMID:32674113